positive regulation of nitrogen cycle metabolic process [GO:1903316] (biological process) Definition: Any process that activates or increases the frequency, rate or extent of nitrogen cycle metabolic process. Also known as: up regulation of nitrogen cycle metabolic process, up-regulation of nitrogen cycle metabolic process, upregulation of nitrogen cycle metabolic process, activation of nitrogen cycle metabolic process Subtypes: GO:1901714 Relationships: is a type of positive regulation of metabolic process [GO:0009893]; is a type of regulation of nitrogen cycle metabolic process [GO:1903314]; positively regulates nitrogen cycle metabolic process [GO:0071941] Sources: GOC:TermGenie, GOC:vw, GO_REF:0000058